{
  "term_id": "UNKNOWN:0002",
  "term_label": "Unknown biological process",
  "gene_symbol": "TRAJ38",
  "gene": "UniProtKB:A0A075B6W7",
  "gene_name": "T cell receptor alpha joining 38 (Fragment)"
}